{
  "term_label": "Unknown cellular component",
  "gene": "UniProtKB:O95671",
  "gene_name": "Probable bifunctional dTTP_UTP pyrophosphatase_methyltransferase protein",
  "term_id": "UNKNOWN:0003",
  "gene_symbol": "ASMTL"
}